{
  "gene_symbol": "GCGR",
  "gene_name": "Glucagon receptor",
  "gene": "UniProtKB:P47871",
  "term_label": "glucagon receptor activity",
  "term_id": "GO:0004967"
}